{
  "term_id": "GO:0005085",
  "term_label": "guanyl-nucleotide exchange factor activity",
  "gene": "UniProtKB:O15013",
  "gene_symbol": "ARHGEF10",
  "gene_name": "Rho guanine nucleotide exchange factor 10"
}